protein-lipid complex [GO:0032994] (cellular component) Subtypes: lipid tube [GO:0060987], lipoprotein particle [GO:1990777] Note: Macromolecular complexes in which the lipid component is all covalently bound to protein are not considered protein-lipid complexes. Definition: A macromolecular complex containing separate protein and lipid molecules. Separate in this context means not covalently bound to each other. Relationships: is a type of GO:0032991 Sources: GOC:mah